{
  "gene_name": "NACHT, LRR and PYD domains-containing protein 3",
  "gene": "UniProtKB:Q96P20",
  "term_label": "NLRP3 inflammasome complex",
  "term_id": "GO:0072559",
  "gene_symbol": "NLRP3"
}